{
  "term_id": "GO:0032956",
  "gene_name": "Rho-related GTP-binding protein Rho6",
  "term_label": "regulation of actin cytoskeleton organization",
  "gene_symbol": "RND1",
  "gene": "UniProtKB:Q92730"
}